positive regulation of alpha-beta T cell differentiation [GO:0046638] (biological process) Also known as: positive regulation of alpha-beta T lymphocyte differentiation, positive regulation of alpha-beta T-cell differentiation, positive regulation of alpha-beta T-lymphocyte differentiation, up regulation of alpha-beta T cell differentiation, up-regulation of alpha-beta T cell differentiation, upregulation of alpha-beta T cell differentiation, activation of alpha-beta T cell differentiation, stimulation of alpha-beta T cell differentiation, positive regulation of alpha-beta T cell development Relationships: is_a positive regulation of T cell differentiation [GO:0045582]; is_a positive regulation of alpha-beta T cell activation [GO:0046635]; is a type of regulation of alpha-beta T cell differentiation [GO:0046637]; positively regulates alpha-beta T cell differentiation [GO:0046632] Definition: Any process that activates or increases the frequency, rate or extent of alpha-beta T cell differentiation. Note: Note that immunologists typically use the word 'development' to refer to cells of B or T cell lineages undergoing the process that GO describes as 'cell differentiation'. Sources: GOC:ai Subtypes: positive regulation of CD4-positive, alpha-beta T cell differentiation [GO:0043372], positive regulation of CD8-positive, alpha-beta T cell differentiation [GO:0043378], positive regulation of NK T cell differentiation [GO:0051138]